{
  "gene": "UniProtKB:Q02809",
  "term_label": "procollagen-lysine 5-dioxygenase activity",
  "gene_name": "Procollagen-lysine,2-oxoglutarate 5-dioxygenase 1",
  "gene_symbol": "PLOD1",
  "term_id": "GO:0008475"
}